{
  "gene_symbol": "DSPP",
  "gene_name": "Dentin sialophosphoprotein",
  "term_label": "odontoblast differentiation",
  "term_id": "GO:0071895",
  "gene": "UniProtKB:Q9NZW4"
}